{
  "term_id": "UNKNOWN:0002",
  "gene_symbol": "DEFB124",
  "term_label": "Unknown biological process",
  "gene_name": "Beta-defensin 124",
  "gene": "UniProtKB:Q8NES8"
}